{
  "gene": "UniProtKB:Q92889",
  "gene_symbol": "ERCC4",
  "gene_name": "DNA repair endonuclease XPF",
  "term_label": "double-strand break repair via homologous recombination",
  "term_id": "GO:0000724"
}